{
  "gene": "UniProtKB:O43246",
  "gene_symbol": "SLC7A4",
  "term_id": "GO:0006865",
  "gene_name": "Cationic amino acid transporter 4",
  "term_label": "amino acid transport"
}